{
  "gene_symbol": "CNTN6",
  "gene": "UniProtKB:Q9UQ52",
  "term_label": "homophilic cell-cell adhesion",
  "gene_name": "Contactin-6",
  "term_id": "GO:0007156"
}